maintenance of plant organ identity [GO:0090700] (BP) Subtypes: maintenance of floral organ identity [GO:0048497] Definition: The process in which the identity of a plant organ is maintained. Identity is considered to be the aggregate of characteristics by which a structure is recognized. References: PMID:9090883 Sources: GOC:tb Relationships: is a type of negative regulation of cell differentiation [GO:0045596]; is part of plant organ development [GO:0099402]